{
  "gene_name": "ADP-ribosylation factor-like protein 15",
  "term_id": "UNKNOWN:0001",
  "term_label": "Unknown molecular function",
  "gene": "UniProtKB:Q9NXU5",
  "gene_symbol": "ARL15"
}